{
  "gene_name": "Tyrosine-protein phosphatase non-receptor type 1",
  "term_id": "GO:0005783",
  "gene": "UniProtKB:P18031",
  "gene_symbol": "PTPN1",
  "term_label": "endoplasmic reticulum"
}